filamentous growth [GO:0030447] (BP) Regulation: regulated by regulation of filamentous growth [GO:0010570]; negatively regulated by negative regulation of filamentous growth [GO:0060258]; positively regulated by GO:0090033 Relationships: is a type of GO:0040007 Definition: The process in which a multicellular organism, a unicellular organism or a group of unicellular organisms grow in a threadlike, filamentous shape. References: PMID:11729141 Sources: GOC:mcc Subtypes: hyphal growth [GO:0030448], filamentous growth of a unicellular organism [GO:0044180], GO:0044181, GO:0044182